{
  "gene_symbol": "ADPRH",
  "term_id": "UNKNOWN:0003",
  "term_label": "Unknown cellular component",
  "gene_name": "ADP-ribosylhydrolase ARH1",
  "gene": "UniProtKB:P54922"
}